{
  "gene_name": "Zinc finger protein 17",
  "term_label": "DNA-binding transcription factor activity, RNA polymerase II-specific",
  "term_id": "GO:0000981",
  "gene_symbol": "ZNF17",
  "gene": "UniProtKB:P17021"
}